{
  "gene_name": "Bifunctional heparan sulfate N-deacetylase_N-sulfotransferase 2",
  "gene": "UniProtKB:P52849",
  "term_id": "GO:0019213",
  "gene_symbol": "NDST2",
  "term_label": "deacetylase activity"
}